{
  "term_id": "GO:0001578",
  "gene_symbol": "TPPP3",
  "gene": "UniProtKB:Q9BW30",
  "term_label": "microtubule bundle formation",
  "gene_name": "Tubulin polymerization-promoting protein family member 3"
}